{
  "gene": "UniProtKB:Q9NZP6",
  "term_label": "nuclear pore",
  "gene_name": "Nuclear pore-associated protein 1",
  "gene_symbol": "NPAP1",
  "term_id": "GO:0005643"
}